{
  "gene_symbol": "MAGEB16",
  "gene_name": "Melanoma-associated antigen B16",
  "gene": "UniProtKB:A2A368",
  "term_id": "GO:0005634",
  "term_label": "nucleus"
}